{
  "gene_name": "Protein mono-ADP-ribosyltransferase PARP4",
  "gene_symbol": "PARP4",
  "gene": "UniProtKB:Q9UKK3",
  "term_label": "Unknown biological process",
  "term_id": "UNKNOWN:0002"
}